{
  "gene_name": "CREB-regulated transcription coactivator 3",
  "term_label": "transcription coactivator activity",
  "gene": "UniProtKB:Q6UUV7",
  "gene_symbol": "CRTC3",
  "term_id": "GO:0003713"
}